positive regulation of phosphate transmembrane transport [GO:2000187] (BP) Relationships: is a type of GO:0034764; is a type of regulation of phosphate transmembrane transport [GO:2000185]; positively regulates GO:0035435 Sources: GOC:obol Definition: Any process that activates or increases the frequency, rate or extent of phosphate transmembrane transport. Also known as: positive regulation of phosphate membrane transport